positive regulation of intrinsic apoptotic signaling pathway in response to DNA damage [GO:1902231] (biological process) Definition: Any process that activates or increases the frequency, rate or extent of intrinsic apoptotic signaling pathway in response to DNA damage. Relationships: is a type of regulation of intrinsic apoptotic signaling pathway in response to DNA damage [GO:1902229]; is a type of GO:2001244; positively regulates GO:0008630 Subtypes: GO:1902167 References: PMID:15314165 Sources: GOC:BHF, GOC:TermGenie, GOC:mtg_apoptosis, GOC:rl Also known as: up regulation of intrinsic apoptotic signaling pathway in response to DNA damage, up-regulation of intrinsic apoptotic signaling pathway in response to DNA damage, upregulation of intrinsic apoptotic signaling pathway in response to DNA damage, activation of intrinsic apoptotic signaling pathway in response to DNA damage, activation of DNA damage response, signal transduction resulting in induction of apoptosis, positive regulation of DNA damage response, signal transduction resulting in induction of apoptosis, up regulation of DNA damage response, signal transduction resulting in induction of apoptosis, up-regulation of DNA damage response, signal transduction resulting in induction of apoptosis, upregulation of DNA damage response, signal transduction resulting in induction of apoptosis